{
  "gene_symbol": "CDH2",
  "term_id": "GO:0000902",
  "term_label": "cell morphogenesis",
  "gene": "UniProtKB:P19022",
  "gene_name": "Cadherin-2"
}